defecation rhythm [GO:0035882] (BP) References: PMID:7479775, PMID:8158250, PMID:9066270 Sources: GOC:bf, GOC:kmv Definition: The rhythmic process of defecation that consists of an intestinal oscillator which regulates calcium waves. These waves in turn control a stereotypical, three-part pattern of muscle contractions. In some organisms, defecation can recur with a regularity more frequent than every 24 hours. For example, in a well-fed Caenorhabditis elegans, the defecation motor program occurs approximately every 45 seconds, and is temperature- and touch-compensated. Also known as: DMP, defecation cycle, defecation motor program, defecation behavior Regulation: regulated by GO:2000746; negatively regulated by negative regulation of defecation rhythm [GO:2000747]; positively regulated by positive regulation of defecation rhythm [GO:2000748] Relationships: is a type of ultradian rhythm [GO:0007624]; is part of defecation [GO:0030421]